{
  "term_id": "GO:0050852",
  "term_label": "T cell receptor signaling pathway",
  "gene": "UniProtKB:O00478",
  "gene_symbol": "BTN3A3",
  "gene_name": "Butyrophilin subfamily 3 member A3"
}